glutathione biosynthetic process [GO:0006750] (biological process) Regulation: RO_0002211 by regulation of glutathione biosynthetic process [GO:1903786]; negatively regulated by negative regulation of glutathione biosynthetic process [GO:1903787]; positively regulated by GO:1903788 Sources: GOC:ai, GOC:al, GOC:pde, ISBN:0198506732 Relationships: is a type of glutathione metabolic process [GO:0006749]; is a type of GO:0019184; is_a GO:0042398; is a type of amide biosynthetic process [GO:0043604]; is a type of sulfur compound biosynthetic process [GO:0044272] Also known as: glutathione anabolism, glutathione biosynthesis, glutathione formation, glutathione synthesis Definition: The chemical reactions and pathways resulting in the formation of glutathione, the tripeptide glutamylcysteinylglycine, which acts as a coenzyme for some enzymes and as an antioxidant in the protection of sulfhydryl groups in enzymes and other proteins.